{
  "term_label": "(R)-carnitine transmembrane transporter activity",
  "gene": "UniProtKB:Q9UN76",
  "gene_symbol": "SLC6A14",
  "gene_name": "Sodium- and chloride-dependent neutral and basic amino acid transporter B(0+)",
  "term_id": "GO:1901235"
}